{
  "term_label": "cholesterol homeostasis",
  "gene": "UniProtKB:P02656",
  "gene_symbol": "APOC3",
  "gene_name": "Apolipoprotein C-III",
  "term_id": "GO:0042632"
}